{
  "gene_symbol": "VSTM4",
  "term_id": "UNKNOWN:0002",
  "term_label": "Unknown biological process",
  "gene": "UniProtKB:Q8IW00",
  "gene_name": "V-set and transmembrane domain-containing protein 4"
}